mitochondrial tRNA modification [GO:0070900] (biological process) Sources: GOC:mah, GOC:mcc Subtypes: mitochondrial tRNA wobble uridine modification [GO:0070899], mitochondrial tRNA methylation [GO:0070901], mitochondrial tRNA pseudouridine synthesis [GO:0070902], mitochondrial tRNA thio-modification [GO:0070903], mitochondrial tRNA threonylcarbamoyladenosine modification [GO:0072670] Definition: The covalent alteration of one or more nucleotides within a mitochondrial tRNA molecule to produce a mitochondrial tRNA molecule with a sequence that differs from that coded genetically. Relationships: is a type of tRNA modification [GO:0006400]; is a type of tRNA threonylcarbamoyladenosine metabolic process [GO:0070525]; is a type of GO:0090646; is a type of mitochondrial RNA modification [GO:1900864]